{
  "gene": "UniProtKB:A0A1W2PRN6",
  "term_id": "GO:0051123",
  "gene_name": "HCG1807616",
  "term_label": "RNA polymerase II preinitiation complex assembly",
  "gene_symbol": "LINC02218"
}